{
  "gene": "UniProtKB:P45379",
  "term_label": "tropomyosin binding",
  "term_id": "GO:0005523",
  "gene_name": "Troponin T, cardiac muscle",
  "gene_symbol": "TNNT2"
}